lipid tube [GO:0060987] (CC) Definition: A macromolecular complex that contains a tube of lipid surrounded by a protein coat. Relationships: is a type of protein-lipid complex [GO:0032994] Sources: GOC:ascb_2009, GOC:dph, GOC:tb